{
  "gene_name": "Cathepsin L2",
  "term_id": "GO:0004197",
  "gene": "UniProtKB:O60911",
  "gene_symbol": "CTSV",
  "term_label": "cysteine-type endopeptidase activity"
}